{
  "gene_name": "Glypican-1",
  "gene": "UniProtKB:P35052",
  "gene_symbol": "GPC1",
  "term_id": "GO:0045202",
  "term_label": "synapse"
}